{
  "gene": "UniProtKB:Q9HAD4",
  "term_id": "UNKNOWN:0002",
  "term_label": "Unknown biological process",
  "gene_symbol": "WDR41",
  "gene_name": "WD repeat-containing protein 41"
}